{
  "gene_symbol": "ITGB3",
  "term_id": "GO:0005925",
  "gene": "UniProtKB:P05106",
  "term_label": "focal adhesion",
  "gene_name": "Integrin beta-3"
}